{
  "gene": "UniProtKB:Q6DN72",
  "term_label": "cell surface receptor signaling pathway",
  "gene_name": "Fc receptor-like protein 6",
  "gene_symbol": "FCRL6",
  "term_id": "GO:0007166"
}